{
  "term_label": "glycine biosynthetic process from serine",
  "term_id": "GO:0019264",
  "gene_symbol": "SHMT2",
  "gene_name": "Serine hydroxymethyltransferase, mitochondrial",
  "gene": "UniProtKB:P34897"
}